{
  "gene_name": "Heme transporter FLVCR2",
  "gene_symbol": "FLVCR2",
  "term_label": "heme export",
  "gene": "UniProtKB:Q9UPI3",
  "term_id": "GO:0097037"
}